{
  "term_label": "helicase activity",
  "gene_name": "Probable ATP-dependent RNA helicase DHX35",
  "term_id": "GO:0004386",
  "gene_symbol": "DHX35",
  "gene": "UniProtKB:Q9H5Z1"
}